{
  "gene": "UniProtKB:Q9NR31",
  "term_label": "GTPase activity",
  "term_id": "GO:0003924",
  "gene_name": "GTP-binding protein SAR1a",
  "gene_symbol": "SAR1A"
}